{
  "term_id": "GO:0006357",
  "gene_name": "T-box transcription factor TBX22",
  "gene_symbol": "TBX22",
  "gene": "UniProtKB:Q9Y458",
  "term_label": "regulation of transcription by RNA polymerase II"
}